{
  "gene_symbol": "NAP1L6P",
  "gene": "UniProtKB:A6NFF2",
  "gene_name": "Putative nucleosome assembly protein 1-like 6",
  "term_label": "Unknown cellular component",
  "term_id": "UNKNOWN:0003"
}